{
  "gene": "UniProtKB:Q9UI10",
  "gene_symbol": "EIF2B4",
  "gene_name": "Translation initiation factor eIF-2B subunit delta",
  "term_label": "eukaryotic translation initiation factor 2B complex",
  "term_id": "GO:0005851"
}